{
  "gene": "UniProtKB:A0A075B704",
  "term_label": "Unknown cellular component",
  "term_id": "UNKNOWN:0003",
  "gene_name": "T cell receptor alpha joining 57 (Fragment)",
  "gene_symbol": "TRAJ57"
}